{
  "gene": "UniProtKB:P21980",
  "gene_name": "Protein-glutamine gamma-glutamyltransferase 2",
  "term_id": "GO:0003810",
  "gene_symbol": "TGM2",
  "term_label": "protein-glutamine gamma-glutamyltransferase activity"
}